NAD+ biosynthetic process via the salvage pathway [GO:0034355] (biological process) Definition: The chemical reactions and pathways resulting in the formation of nicotinamide-adenine dinucleotide (NAD+) from vitamin B3 derivatives (including nicotinic acid (NA) and nicotinamide (NAM)), beta-nicotinamide D-ribonucleotide (NMN), nicotinamide riboside (NR) or nicotinate riboside (NAR), without de novo synthesis. References: PMID:12648681, PMID:27374990 Sources: GOC:sjm Also known as: NAD biosynthetic process via the salvage pathway, NAD salvage, NAD salvage pathway Relationships: is a type of NAD+ biosynthetic process [GO:0009435]; is_a GO:0019365; is a type of purine nucleotide salvage [GO:0032261]